{
  "gene_name": "DEP domain-containing protein 7",
  "gene_symbol": "DEPDC7",
  "term_id": "UNKNOWN:0002",
  "term_label": "Unknown biological process",
  "gene": "UniProtKB:Q96QD5"
}